{
  "gene_name": "Ankyrin repeat and SOCS box protein 13",
  "gene": "UniProtKB:Q8WXK3",
  "term_id": "UNKNOWN:0002",
  "gene_symbol": "ASB13",
  "term_label": "Unknown biological process"
}